{
  "term_id": "GO:0046755",
  "gene_name": "Multivesicular body subunit 12B",
  "gene_symbol": "MVB12B",
  "gene": "UniProtKB:Q9H7P6",
  "term_label": "viral budding"
}